post-chaperonin tubulin folding pathway [GO:0007023] (biological process) Definition: Completion of folding of alpha- and beta-tubulin; takes place subsequent to chaperonin-mediated partial folding; mediated by a complex of folding cofactors. References: PMID:10542094 Relationships: is a type of GO:0006457